{
  "gene_name": "Zinc finger protein ubi-d4",
  "gene": "UniProtKB:Q92785",
  "term_label": "transcription coregulator activity",
  "term_id": "GO:0003712",
  "gene_symbol": "DPF2"
}